response to amyloid-beta [GO:1904645] (biological process) Also known as: response to beta-amyloid, response to beta-amyloids Definition: Any process that results in a change in state or activity of a cell or an organism (in terms of movement, secretion, enzyme production, gene expression, etc.) as a result of a amyloid-beta stimulus. Subtypes: cellular response to amyloid-beta [GO:1904646] References: PMID:23555824 Sources: GOC:TermGenie, GO_REF:0000071 Relationships: is a type of response to nitrogen compound [GO:1901698]; is a type of GO:1901700